{
  "gene_name": "HLA class II histocompatibility antigen, DO alpha chain",
  "gene": "UniProtKB:P06340",
  "gene_symbol": "HLA-DOA",
  "term_id": "GO:0023026",
  "term_label": "MHC class II protein complex binding"
}